{
  "gene": "UniProtKB:Q5MNZ9",
  "gene_symbol": "WIPI1",
  "term_label": "nucleophagy",
  "term_id": "GO:0044804",
  "gene_name": "WD repeat domain phosphoinositide-interacting protein 1"
}